{
  "gene": "UniProtKB:P12757",
  "gene_name": "Ski-like protein",
  "gene_symbol": "SKIL",
  "term_id": "GO:0046332",
  "term_label": "SMAD binding"
}